{
  "gene_symbol": "FGD3",
  "term_id": "GO:0005737",
  "term_label": "cytoplasm",
  "gene_name": "FYVE, RhoGEF and PH domain-containing protein 3",
  "gene": "UniProtKB:Q5JSP0"
}